{
  "term_id": "UNKNOWN:0003",
  "gene": "UniProtKB:Q8IXS0",
  "gene_name": "Protein FAM217A",
  "term_label": "Unknown cellular component",
  "gene_symbol": "FAM217A"
}